compartment boundary maintenance [GO:0060289] (biological process) Sources: GOC:dph Relationships: is a type of tissue homeostasis [GO:0001894]; is part of compartment pattern specification [GO:0007386] Definition: A homeostatic process involved in the maintenance of a compartment boundary. A compartment boundary is a lineage restriction boundary within a developing tissue which does not correspond to some morphological barrier.